FAD binding [GO:0071949] (molecular function) Also known as: oxidized flavin adenine dinucleotide binding, oxidized flavine-adenine dinucleotide binding Definition: Binding to the oxidized form, FAD, of flavin-adenine dinucleotide, the coenzyme or the prosthetic group of various flavoprotein oxidoreductase enzymes. Relationships: is a type of flavin adenine dinucleotide binding [GO:0050660] Sources: GOC:mah